{
  "term_label": "ceramide biosynthetic process",
  "gene_name": "Sphingomyelin phosphodiesterase 4",
  "gene": "UniProtKB:Q9NXE4",
  "gene_symbol": "SMPD4",
  "term_id": "GO:0046513"
}